{
  "gene_symbol": "EXOC1",
  "term_label": "exocyst",
  "term_id": "GO:0000145",
  "gene": "UniProtKB:Q9NV70",
  "gene_name": "Exocyst complex component 1"
}